{
  "gene_symbol": "SCNN1A",
  "gene": "UniProtKB:P37088",
  "term_id": "GO:0005886",
  "gene_name": "Amiloride-sensitive sodium channel subunit alpha",
  "term_label": "plasma membrane"
}